sphingosine kinase activity [GO:0008481] (molecular function) Definition: Catalysis of the reaction: a sphingoid base + ATP = a sphingoid 1-phosphate + ADP + H+. Sources: RHEA:51496 Also known as: ATP:sphinganine 1-phosphotransferase activity, dihydrosphingosine kinase (phosphorylating), dihydrosphingosine kinase activity, sphinganine kinase activity, sphingosine kinase (phosphorylating) Relationships: is_a GO:0001727; is a type of GO:0016773